ribonuclease IV activity [GO:0033893] (molecular function) Relationships: is a type of RNA endonuclease activity producing 5'-phosphomonoesters, hydrolytic mechanism [GO:0016891] Definition: Catalysis of the endonucleolytic cleavage of poly(A) to fragments terminated by 3'-hydroxy and 5'-phosphate groups. Also known as: endoribonuclease IV activity Sources: EC:3.1.26.6